{
  "gene_name": "Visual system homeobox 1",
  "term_id": "GO:0000976",
  "term_label": "transcription cis-regulatory region binding",
  "gene_symbol": "VSX1",
  "gene": "UniProtKB:Q9NZR4"
}